{
  "gene_name": "Histidine protein methyltransferase 1 homolog",
  "term_label": "regulation of translation",
  "term_id": "GO:0006417",
  "gene": "UniProtKB:O95568",
  "gene_symbol": "METTL18"
}